{
  "gene_symbol": "LAMA5",
  "gene_name": "Laminin subunit alpha-5",
  "gene": "UniProtKB:O15230",
  "term_label": "extracellular matrix structural constituent",
  "term_id": "GO:0005201"
}